glucosidase activity [GO:0015926] (molecular function) Relationships: is a type of hydrolase activity, hydrolyzing O-glycosyl compounds [GO:0004553] Definition: Catalysis of the hydrolysis of glucosyl compounds, substances containing a group derived from a cyclic form of glucose or a glucose derivative. Subtypes: beta-glucosidase activity [GO:0008422], protein-glucosylgalactosylhydroxylysine glucosidase activity [GO:0047402], 2-deoxyglucosidase activity [GO:0047539], GDP-glucosidase activity [GO:0047917], maltose-6'-phosphate glucosidase activity [GO:0050081], alpha-glucosidase activity [GO:0090599] Sources: ISBN:0198506732